{
  "term_label": "nucleus",
  "gene_symbol": "CYREN",
  "gene": "UniProtKB:Q9BWK5",
  "term_id": "GO:0005634",
  "gene_name": "Cell cycle regulator of non-homologous end joining"
}